{
  "gene_name": "Protein RER1",
  "term_id": "GO:0000139",
  "gene": "UniProtKB:O15258",
  "term_label": "Golgi membrane",
  "gene_symbol": "RER1"
}